D-tryptophan N-acetyltransferase activity [GO:0047835] (molecular function) Also known as: D-tryptophan acetyltransferase activity, acetyl-CoA-D-tryptophan-alpha-N-acetyltransferase activity, acetyl-CoA:D-tryptophan N-acetyltransferase activity Sources: RHEA:10060 Definition: Catalysis of the reaction: D-tryptophan + acetyl-CoA = N-acetyl-D-tryptophan + CoA + H+. Relationships: is_a D-amino-acid N-acetyltransferase activity [GO:0047812]